negative regulation of mast cell degranulation [GO:0043305] (biological process) Also known as: down regulation of mast cell degranulation, down-regulation of mast cell degranulation, downregulation of mast cell degranulation, negative regulation of mast cell granule exocytosis, inhibition of mast cell degranulation Relationships: is a type of negative regulation of myeloid leukocyte mediated immunity [GO:0002887]; is a type of negative regulation of leukocyte degranulation [GO:0043301]; is a type of regulation of mast cell degranulation [GO:0043304]; negatively regulates mast cell degranulation [GO:0043303] Sources: ISBN:0781735149 Definition: Any process that stops, prevents, or reduces the rate of mast cell degranulation.